{
  "term_label": "regulation of bone remodeling",
  "gene_name": "SUN domain-containing ossification factor",
  "gene": "UniProtKB:Q9UBS9",
  "gene_symbol": "SUCO",
  "term_id": "GO:0046850"
}